{
  "gene_symbol": "LRRC4",
  "gene_name": "Leucine-rich repeat-containing protein 4",
  "gene": "UniProtKB:Q9HBW1",
  "term_id": "GO:0098839",
  "term_label": "postsynaptic density membrane"
}